mandelate racemase activity [GO:0018838] (molecular function) Relationships: is a type of racemase and epimerase activity, acting on hydroxy acids and derivatives [GO:0016856] Definition: Catalysis of the reaction: (S)-mandelate = (R)-mandelate. Sources: EC:5.1.2.2